positive regulation of blood vessel branching [GO:1905555] (BP) Also known as: positive regulation of branching involved in blood vessel morphogenesis, up regulation of branching involved in blood vessel morphogenesis, up regulation of patterning of blood vessels, up-regulation of branching involved in blood vessel morphogenesis, up-regulation of patterning of blood vessels, upregulation of branching involved in blood vessel morphogenesis, upregulation of patterning of blood vessels, activation of branching involved in blood vessel morphogenesis, activation of patterning of blood vessels Definition: Any process that activates or increases the frequency, rate or extent of blood vessel branching. Relationships: is a type of positive regulation of angiogenesis [GO:0045766]; is a type of positive regulation of morphogenesis of an epithelium [GO:1905332]; is a type of regulation of blood vessel branching [GO:1905553]; RO_0002213 branching involved in blood vessel morphogenesis [GO:0001569] References: PMID:23201774 Sources: GOC:BHF, GOC:BHF_telomere, GOC:TermGenie, GOC:nc, GO_REF:0000058